{
  "term_label": "transmembrane receptor protein tyrosine kinase activity",
  "gene_name": "Angiopoietin-1 receptor",
  "term_id": "GO:0004714",
  "gene_symbol": "TEK",
  "gene": "UniProtKB:Q02763"
}